[cytochrome c]-methionine S-methyltransferase activity [GO:0030783] (molecular function) Sources: EC:2.1.1.123 Relationships: is a type of S-adenosylmethionine-dependent methyltransferase activity [GO:0008757] Also known as: S-adenosyl-L-methionine:cytochrome c-methionine S-methyltransferase activity, cytochrome c-methionine S-methyltransferase activity Definition: Catalysis of the reaction: S-adenosyl-L-methionine + [cytochrome c]-methionine = S-adenosyl-L-homocysteine + [cytochrome c]-S-methyl-methionine.